dibenzothiophene desulfurization [GO:0018897] (BP) Definition: The removal of the sulfur atom from dibenzothiophene, a substance composed of two benzene rings linked by one sulfide bond and one carbon-carbon bond. Also known as: dibenzothiophene desulphurization Sources: GOC:ai Relationships: is a type of GO:0042178